{
  "gene_name": "Zinc finger protein 532",
  "term_label": "Unknown molecular function",
  "term_id": "UNKNOWN:0001",
  "gene": "UniProtKB:Q9HCE3",
  "gene_symbol": "ZNF532"
}